{
  "gene_symbol": "NBPF8",
  "term_id": "UNKNOWN:0002",
  "gene_name": "Putative neuroblastoma breakpoint family member 8",
  "term_label": "Unknown biological process",
  "gene": "UniProtKB:Q3BBV2"
}